{
  "gene": "UniProtKB:P15509",
  "term_id": "GO:0005829",
  "gene_name": "Granulocyte-macrophage colony-stimulating factor receptor subunit alpha",
  "term_label": "cytosol",
  "gene_symbol": "CSF2RA"
}